{
  "term_id": "GO:0005654",
  "gene": "UniProtKB:P54727",
  "gene_symbol": "RAD23B",
  "gene_name": "UV excision repair protein RAD23 homolog B",
  "term_label": "nucleoplasm"
}